{
  "term_label": "cytoplasm",
  "gene_name": "SR-related and CTD-associated factor 8",
  "gene": "UniProtKB:Q9UPN6",
  "term_id": "GO:0005737",
  "gene_symbol": "SCAF8"
}